{
  "gene_symbol": "MAGI1",
  "gene": "UniProtKB:Q96QZ7",
  "gene_name": "Membrane-associated guanylate kinase, WW and PDZ domain-containing protein 1",
  "term_label": "signal transduction",
  "term_id": "GO:0007165"
}